{
  "gene_name": "Thiosulfate:glutathione sulfurtransferase",
  "gene": "UniProtKB:Q8NFU3",
  "term_label": "Unknown molecular function",
  "gene_symbol": "TSTD1",
  "term_id": "UNKNOWN:0001"
}